{
  "term_id": "GO:0014839",
  "term_label": "myoblast migration involved in skeletal muscle regeneration",
  "gene_symbol": "AKIRIN1",
  "gene": "UniProtKB:Q9H9L7",
  "gene_name": "Akirin-1"
}